{
  "term_id": "GO:0070328",
  "gene_symbol": "GPIHBP1",
  "term_label": "triglyceride homeostasis",
  "gene": "UniProtKB:Q8IV16",
  "gene_name": "Glycosylphosphatidylinositol-anchored high density lipoprotein-binding protein 1"
}